{
  "term_label": "actin binding",
  "gene_symbol": "SYNPO2",
  "term_id": "GO:0003779",
  "gene_name": "Synaptopodin-2",
  "gene": "UniProtKB:Q9UMS6"
}